{
  "gene_symbol": "XRCC2",
  "term_id": "GO:0033063",
  "term_label": "Rad51B-Rad51C-Rad51D-XRCC2 complex",
  "gene": "UniProtKB:O43543",
  "gene_name": "DNA repair protein XRCC2"
}